8-hydroxy-dADP phosphatase activity [GO:0044717] (molecular function) References: PMID:22556419 Sources: GOC:pde Relationships: is a type of GO:0017110 Definition: Catalysis of the reaction: 8-hydroxy-dADP + H2O = 8-hydroxy-dAMP + phosphate.